{
  "gene": "UniProtKB:Q5D1E8",
  "term_label": "mRNA binding",
  "term_id": "GO:0003729",
  "gene_name": "Endoribonuclease ZC3H12A",
  "gene_symbol": "ZC3H12A"
}